{
  "term_id": "UNKNOWN:0001",
  "gene": "UniProtKB:Q2T9L4",
  "gene_symbol": "INSYN1",
  "term_label": "Unknown molecular function",
  "gene_name": "Inhibitory synaptic factor 1"
}